{
  "gene_symbol": "OR9G4",
  "gene": "UniProtKB:Q8NGQ1",
  "gene_name": "Olfactory receptor 9G4",
  "term_id": "GO:0007608",
  "term_label": "sensory perception of smell"
}